{
  "term_label": "glutathione peroxidase activity",
  "term_id": "GO:0004602",
  "gene": "UniProtKB:Q99735",
  "gene_name": "Microsomal glutathione S-transferase 2",
  "gene_symbol": "MGST2"
}